threonine efflux transmembrane transporter activity [GO:0015565] (molecular function) Also known as: threonine efflux permease activity, threonine export transporter activity, threonine export protein Sources: GOC:mtg_transport, ISBN:0815340729 Definition: Enables the transfer of threonine from the inside of the cell to the outside of the cell across a membrane. Relationships: is a type of GO:0015195; is a type of GO:0034639